{
  "term_label": "Unknown cellular component",
  "term_id": "UNKNOWN:0003",
  "gene_name": "Zinc finger protein 257",
  "gene": "UniProtKB:Q9Y2Q1",
  "gene_symbol": "ZNF257"
}